camera-type eye morphogenesis [GO:0048593] (biological process) Also known as: camera-style eye morphogenesis Relationships: is a type of eye morphogenesis [GO:0048592]; is part of GO:0043010 Definition: The process in which the anatomical structures of the eye are generated and organized. The camera-type eye is an organ of sight that receives light through an aperture and focuses it through a lens, projecting it on a photoreceptor field. Sources: GOC:jid, GOC:mtg_sensu